macrophage activation involved in immune response [GO:0002281] (biological process) Definition: A change in morphology and behavior of a macrophage resulting from exposure to a cytokine, chemokine, cellular ligand, or soluble factor, leading to the initiation or perpetuation of an immune response. Also known as: macrophage polarization involved in immune response, macrophage activation during immune response Sources: GOC:add, ISBN:0781735149 Subtypes: GO:0002282 Relationships: is a type of leukocyte activation involved in immune response [GO:0002366]; is a type of macrophage activation [GO:0042116]; BFO_0000050 myeloid cell activation involved in immune response [GO:0002275]